{
  "term_id": "GO:1904047",
  "term_label": "S-adenosyl-L-methionine binding",
  "gene": "UniProtKB:Q14749",
  "gene_symbol": "GNMT",
  "gene_name": "Glycine N-methyltransferase"
}